urinary bladder smooth muscle contraction [GO:0014832] (biological process) Subtypes: GO:0060083 Relationships: is a type of urinary tract smooth muscle contraction [GO:0014848] References: PMID:11768524, PMID:18276178, PMID:538956 Sources: GOC:mr, GOC:mtg_muscle Definition: A process in which force is generated within smooth muscle tissue, resulting in a change in muscle geometry. This process occurs in the urinary bladder. Force generation involves a chemo-mechanical energy conversion step that is carried out by the actin/myosin complex activity, which generates force through ATP hydrolysis. The urinary bladder is a musculomembranous sac along the urinary tract.